lysine dehydrogenase activity [GO:0050069] (molecular function) Sources: EC:1.4.1.15, MetaCyc:LYSINE-DEHYDROGENASE-RXN Relationships: is a type of oxidoreductase activity, acting on the CH-NH2 group of donors, NAD or NADP as acceptor [GO:0016639] Definition: Catalysis of the reaction: L-lysine + NAD+ = 1,2-didehydropiperidine-2-carboxylate + NH3 + NADH. Also known as: L-lysine:NAD+ oxidoreductase (deaminating, cyclizing)